positive regulation of mitotic sister chromatid arm separation [GO:1905824] (BP) Relationships: is a type of positive regulation of mitotic sister chromatid separation [GO:1901970]; is a type of regulation of mitotic sister chromatid arm separation [GO:1905822]; RO_0002213 mitotic sister chromatid arm separation [GO:1990891] Also known as: up regulation of mitotic sister chromatid arm separation, up-regulation of mitotic sister chromatid arm separation, upregulation of mitotic sister chromatid arm separation, activation of mitotic sister chromatid arm separation References: PMID:18765790 Sources: GOC:TermGenie, GOC:als, GO_REF:0000058 Definition: Any process that activates or increases the frequency, rate or extent of mitotic sister chromatid arm separation.